cellular response to lipopolysaccharide [GO:0071222] (biological process) Definition: Any process that results in a change in state or activity of a cell (in terms of movement, secretion, enzyme production, gene expression, etc.) as a result of a lipopolysaccharide stimulus; lipopolysaccharide is a major component of the cell wall of gram-negative bacteria. Relationships: is a type of response to lipopolysaccharide [GO:0032496]; is a type of GO:0071219; is a type of GO:0071396; is a type of cellular response to oxygen-containing compound [GO:1901701] Also known as: cellular response to endotoxin, cellular response to LPS Sources: GOC:mah